{
  "gene_name": "Protein phosphatase 1 regulatory subunit 14A",
  "gene_symbol": "PPP1R14A",
  "gene": "UniProtKB:Q96A00",
  "term_id": "UNKNOWN:0002",
  "term_label": "Unknown biological process"
}